{
  "gene": "UniProtKB:Q9Y5W3",
  "gene_symbol": "KLF2",
  "gene_name": "Krueppel-like factor 2",
  "term_label": "RNA polymerase II cis-regulatory region sequence-specific DNA binding",
  "term_id": "GO:0000978"
}